{
  "gene_symbol": "CHAC1",
  "gene_name": "Glutathione-specific gamma-glutamylcyclotransferase 1",
  "gene": "UniProtKB:Q9BUX1",
  "term_id": "GO:0005737",
  "term_label": "cytoplasm"
}